hydroxymandelonitrile glucosyltransferase activity [GO:0047239] (molecular function) Definition: Catalysis of the reaction: 4-hydroxymandelonitrile + UDP-D-glucose = H+ + taxiphyllin + UDP. Sources: EC:2.4.1.178, RHEA:15961 Also known as: UDP-glucose:4-hydroxymandelonitrile glucosyltransferase activity, UDPglucose:4-hydroxymandelonitrile glucosyltransferase activity, cyanohydrin glucosyltransferase activity Relationships: is_a UDP-glucosyltransferase activity [GO:0035251]